{
  "term_id": "GO:0042632",
  "term_label": "cholesterol homeostasis",
  "gene": "UniProtKB:Q13133",
  "gene_symbol": "NR1H3",
  "gene_name": "Oxysterols receptor LXR-alpha"
}